{
  "gene": "UniProtKB:Q6ZVW7",
  "gene_name": "Putative interleukin-17 receptor E-like",
  "gene_symbol": "IL17REL",
  "term_label": "Unknown cellular component",
  "term_id": "UNKNOWN:0003"
}